fungiform papilla morphogenesis [GO:0061197] (biological process) Definition: The process in which the anatomical structures of the fungiform papilla are generated and organized. The fungiform papilla is a mushroom-shaped papilla of the tongue. Relationships: is a type of anatomical structure morphogenesis [GO:0009653]; is part of tongue morphogenesis [GO:0043587]; is part of fungiform papilla development [GO:0061196] Sources: GOC:dph